{
  "gene_symbol": "MSH5",
  "term_label": "nucleus",
  "gene_name": "MutS protein homolog 5",
  "term_id": "GO:0005634",
  "gene": "UniProtKB:O43196"
}